{
  "gene": "UniProtKB:Q9UBS4",
  "term_id": "GO:0051787",
  "term_label": "misfolded protein binding",
  "gene_name": "DnaJ homolog subfamily B member 11",
  "gene_symbol": "DNAJB11"
}